type-III dockerin domain binding [GO:1990310] (molecular function) References: PMID:23195689, PMID:24080387 Sources: GOC:mengo_curators Relationships: is a type of GO:0019904 Definition: Binding to a type-III dockerin domain of a protein. Type-III dockerin domain is the binding partner of type-III cohesin domain.